hypoxanthine metabolic process [GO:0046100] (biological process) Also known as: hypoxanthine metabolism Sources: GOC:go_curators Relationships: is a type of purine nucleobase metabolic process [GO:0006144] Definition: The chemical reactions and pathways involving hypoxanthine, 6-hydroxy purine, an intermediate in the degradation of adenylate. Its ribonucleoside is known as inosine and its ribonucleotide as inosinate. Subtypes: hypoxanthine catabolic process [GO:0009114], GO:0046101